{
  "gene_name": "UPF0606 protein KIAA1549L",
  "gene": "UniProtKB:Q6ZVL6",
  "term_id": "UNKNOWN:0002",
  "gene_symbol": "KIAA1549L",
  "term_label": "Unknown biological process"
}